{
  "gene_symbol": "CD22",
  "gene_name": "B-cell receptor CD22",
  "term_label": "recycling endosome",
  "term_id": "GO:0055037",
  "gene": "UniProtKB:P20273"
}